{
  "term_label": "stereocilium tip",
  "term_id": "GO:0032426",
  "gene_name": "Stereocilin",
  "gene": "UniProtKB:Q7RTU9",
  "gene_symbol": "STRC"
}